{
  "term_label": "Hsp70 protein binding",
  "gene": "UniProtKB:P50502",
  "term_id": "GO:0030544",
  "gene_name": "Hsc70-interacting protein",
  "gene_symbol": "ST13"
}